{
  "gene_name": "T cell receptor alpha variable 8-7 (pseudogene) (Fragment)",
  "gene": "UniProtKB:A0A075B6U6",
  "gene_symbol": "TRAV8-7",
  "term_label": "adaptive immune response",
  "term_id": "GO:0002250"
}